{
  "term_label": "protein autoprocessing",
  "term_id": "GO:0016540",
  "gene_name": "Transmembrane protease serine 2",
  "gene_symbol": "TMPRSS2",
  "gene": "UniProtKB:O15393"
}